GTP 3',8'-cyclase activity [GO:0061798] (molecular function) Definition: Catalysis of the reaction: GTP=(8S)-3',8-cyclo-7,8-dihydroguanosine 5'-triphosphate. References: PMID:25896388 Sources: GOC:dph, GOC:ik Relationships: is a type of carbon-carbon lyase activity [GO:0016830]